{
  "term_label": "cytoplasm",
  "gene_name": "Calpain-12",
  "gene": "UniProtKB:Q6ZSI9",
  "term_id": "GO:0005737",
  "gene_symbol": "CAPN12"
}